{
  "term_label": "Unknown cellular component",
  "gene_symbol": "UBE2G1",
  "term_id": "UNKNOWN:0003",
  "gene": "UniProtKB:P62253",
  "gene_name": "Ubiquitin-conjugating enzyme E2 G1"
}